{
  "gene_symbol": "NOS2",
  "term_label": "plasma membrane",
  "term_id": "GO:0005886",
  "gene_name": "Nitric oxide synthase, inducible",
  "gene": "UniProtKB:P35228"
}